phosphoribosyl 1,2-cyclic phosphate 1,2-diphosphodiesterase activity [GO:0102561] (molecular function) Definition: Catalysis of the reaction: alpha-D-ribose 1,2-cyclic phosphate 5-phosphate + H2O = D-ribose 2,5-bisphosphate + H+. Sources: EC:3.1.4.57 Also known as: D-ribose 2,5-bisphosphate 2-phosphohydrolase activity, cyclic phosphate dihydrolase activity Relationships: is a type of phosphoric diester hydrolase activity [GO:0008081]